{
  "gene_symbol": "BAHD1",
  "term_id": "GO:0045892",
  "gene_name": "Bromo adjacent homology domain-containing 1 protein",
  "term_label": "negative regulation of DNA-templated transcription",
  "gene": "UniProtKB:Q8TBE0"
}